{
  "gene": "UniProtKB:Q7Z2D5",
  "term_id": "GO:0007165",
  "term_label": "signal transduction",
  "gene_name": "Phospholipid phosphatase-related protein type 4",
  "gene_symbol": "PLPPR4"
}